{
  "term_id": "GO:0005634",
  "gene_symbol": "SAP30BP",
  "gene": "UniProtKB:Q9UHR5",
  "gene_name": "SAP30-binding protein",
  "term_label": "nucleus"
}